{
  "term_label": "chromosome organization",
  "term_id": "GO:0051276",
  "gene_symbol": "BANF2",
  "gene": "UniProtKB:Q9H503",
  "gene_name": "Barrier-to-autointegration factor-like protein"
}